{
  "gene_symbol": "RPL31",
  "gene": "UniProtKB:P62899",
  "term_label": "cytoplasmic translation",
  "gene_name": "Large ribosomal subunit protein eL31",
  "term_id": "GO:0002181"
}